{
  "term_id": "GO:0005634",
  "term_label": "nucleus",
  "gene_symbol": "HSPB9",
  "gene_name": "Heat shock protein beta-9",
  "gene": "UniProtKB:Q9BQS6"
}